positive regulation of mitotic spindle disassembly [GO:1904687] (biological process) Relationships: is a type of positive regulation of mitotic spindle organization [GO:0110028]; is a type of regulation of mitotic spindle disassembly [GO:1904686]; positively regulates mitotic spindle disassembly [GO:0051228] Definition: Any process that activates or increases the frequency, rate or extent of mitotic spindle disassembly. References: PMID:25963819 Sources: GOC:TermGenie, GO_REF:0000058 Also known as: positive regulation of mitotic spindle breakdown, positive regulation of mitotic spindle catabolism, positive regulation of mitotic spindle degradation, positive regulation of spindle breakdown during mitosis, positive regulation of spindle degradation during mitosis, positive regulation of spindle disassembly during mitosis, up regulation of mitotic spindle breakdown, up regulation of mitotic spindle catabolism, up regulation of mitotic spindle degradation, up regulation of mitotic spindle disassembly, up regulation of spindle breakdown during mitosis, up regulation of spindle degradation during mitosis, up regulation of spindle disassembly during mitosis, up-regulation of mitotic spindle breakdown, up-regulation of mitotic spindle catabolism, up-regulation of mitotic spindle degradation, up-regulation of mitotic spindle disassembly, up-regulation of spindle breakdown during mitosis, up-regulation of spindle degradation during mitosis, up-regulation of spindle disassembly during mitosis, upregulation of mitotic spindle breakdown, upregulation of mitotic spindle catabolism, upregulation of mitotic spindle degradation, upregulation of mitotic spindle disassembly, upregulation of spindle breakdown during mitosis, upregulation of spindle degradation during mitosis, upregulation of spindle disassembly during mitosis, activation of mitotic spindle breakdown, activation of mitotic spindle catabolism, activation of mitotic spindle degradation, activation of mitotic spindle disassembly, activation of spindle breakdown during mitosis, activation of spindle degradation during mitosis, activation of spindle disassembly during mitosis